{
  "gene": "UniProtKB:Q9BXJ4",
  "gene_symbol": "C1QTNF3",
  "gene_name": "Complement C1q tumor necrosis factor-related protein 3",
  "term_id": "GO:0099558",
  "term_label": "maintenance of synapse structure"
}